{
  "gene": "UniProtKB:P50995",
  "gene_name": "Annexin A11",
  "term_id": "GO:0005886",
  "term_label": "plasma membrane",
  "gene_symbol": "ANXA11"
}